{
  "gene": "UniProtKB:Q9NRG4",
  "gene_name": "N-lysine methyltransferase SMYD2",
  "term_label": "histone H3K36 methyltransferase activity",
  "gene_symbol": "SMYD2",
  "term_id": "GO:0046975"
}